{
  "gene_symbol": "DMC1",
  "term_label": "chromosome organization involved in meiotic cell cycle",
  "gene_name": "Meiotic recombination protein DMC1_LIM15 homolog",
  "gene": "UniProtKB:Q14565",
  "term_id": "GO:0070192"
}